peptidyl-proline modification [GO:0018208] (biological process) Definition: The modification of peptidyl-proline. Relationships: is a type of peptidyl-amino acid modification [GO:0018193] Subtypes: GO:0000413, peptidyl-proline hydroxylation [GO:0019511], N-terminal peptidyl-proline methylation [GO:0035568] Sources: GOC:go_curators